{
  "gene_symbol": "MTRNR2L4",
  "term_label": "negative regulation of execution phase of apoptosis",
  "gene_name": "Humanin-like 4",
  "term_id": "GO:1900118",
  "gene": "UniProtKB:P0CJ71"
}